{
  "term_id": "UNKNOWN:0002",
  "gene_name": "TBC1 domain family member 1",
  "gene_symbol": "TBC1D1",
  "gene": "UniProtKB:Q86TI0",
  "term_label": "Unknown biological process"
}